{
  "gene_name": "Protein-lysine N-methyltransferase EEF2KMT",
  "gene": "UniProtKB:Q96G04",
  "gene_symbol": "EEF2KMT",
  "term_label": "protein-lysine N-methyltransferase activity",
  "term_id": "GO:0016279"
}